{
  "term_label": "peptide modification",
  "term_id": "GO:0031179",
  "gene_name": "Putative glutathione hydrolase 3 proenzyme",
  "gene_symbol": "GGT3P",
  "gene": "UniProtKB:A6NGU5"
}